UDP-N-acetyl-alpha-D-fucosamine dehydrogenase activity [GO:0102539] (molecular function) Definition: Catalysis of the reaction: UDP-N-acetyl-alpha-D-fucosamine + NAD(P) = UDP-2-acetamido-4-dehydro-2,6-dideoxy-beta-D-glucose + H+ + NAD(P)H. References: PMID:10627048 Sources: GOC:pz Relationships: is a type of oxidoreductase activity, acting on the CH-OH group of donors, NAD or NADP as acceptor [GO:0016616]